{
  "gene_name": "Trafficking protein particle complex subunit 5",
  "gene": "UniProtKB:Q8IUR0",
  "term_id": "UNKNOWN:0001",
  "gene_symbol": "TRAPPC5",
  "term_label": "Unknown molecular function"
}